response to arsenite(3-) [GO:1903840] (BP) References: PMID:12106899 Sources: GOC:TermGenie, GOC:mr, GO_REF:0000071 Definition: Any process that results in a change in state or activity of a cell or an organism (in terms of movement, secretion, enzyme production, gene expression, etc.) as a result of an arsenite(3-) stimulus. Subtypes: cellular response to arsenite(3-) [GO:1903841] Relationships: is a type of GO:0046685; is a type of response to oxygen-containing compound [GO:1901700]